{
  "gene_name": "von Willebrand factor A domain-containing protein 7",
  "gene": "UniProtKB:Q9Y334",
  "term_id": "UNKNOWN:0002",
  "term_label": "Unknown biological process",
  "gene_symbol": "VWA7"
}